{
  "term_id": "GO:0042428",
  "gene_name": "Amine oxidase [flavin-containing] B",
  "gene_symbol": "MAOB",
  "gene": "UniProtKB:P27338",
  "term_label": "serotonin metabolic process"
}